{
  "gene": "UniProtKB:Q9BYZ6",
  "term_label": "plasma membrane",
  "gene_symbol": "RHOBTB2",
  "gene_name": "Rho-related BTB domain-containing protein 2",
  "term_id": "GO:0005886"
}